{
  "gene_symbol": "ZKSCAN4",
  "term_id": "UNKNOWN:0003",
  "gene_name": "Zinc finger protein with KRAB and SCAN domains 4",
  "gene": "UniProtKB:Q969J2",
  "term_label": "Unknown cellular component"
}